{
  "term_id": "UNKNOWN:0002",
  "term_label": "Unknown biological process",
  "gene": "UniProtKB:O15068",
  "gene_name": "Guanine nucleotide exchange factor DBS",
  "gene_symbol": "MCF2L"
}